{
  "term_id": "GO:0006874",
  "gene": "UniProtKB:Q09013",
  "gene_symbol": "DMPK",
  "term_label": "intracellular calcium ion homeostasis",
  "gene_name": "Myotonin-protein kinase"
}